{
  "term_label": "Unknown cellular component",
  "gene_name": "Intermembrane lipid transfer protein VPS13D",
  "term_id": "UNKNOWN:0003",
  "gene": "UniProtKB:Q5THJ4",
  "gene_symbol": "VPS13D"
}